{
  "gene_name": "Sterol O-acyltransferase 2",
  "gene_symbol": "SOAT2",
  "term_label": "fatty-acyl-CoA binding",
  "term_id": "GO:0000062",
  "gene": "UniProtKB:O75908"
}